{
  "term_id": "UNKNOWN:0001",
  "term_label": "Unknown molecular function",
  "gene_symbol": "TRBV6-7",
  "gene_name": "Probable non-functional T cell receptor beta variable 6-7",
  "gene": "UniProtKB:A0A0A0MS04"
}